{
  "term_id": "GO:0035435",
  "gene_symbol": "SLC37A4",
  "gene": "UniProtKB:O43826",
  "term_label": "phosphate ion transmembrane transport",
  "gene_name": "Glucose-6-phosphate exchanger SLC37A4"
}